{
  "gene_symbol": "KLHL3",
  "gene": "UniProtKB:Q9UH77",
  "gene_name": "Kelch-like protein 3",
  "term_id": "GO:1990756",
  "term_label": "ubiquitin-like ligase-substrate adaptor activity"
}